{
  "gene_symbol": "ARHGAP5",
  "gene_name": "Rho GTPase-activating protein 5",
  "term_label": "GTPase activator activity",
  "gene": "UniProtKB:Q13017",
  "term_id": "GO:0005096"
}